{
  "term_id": "GO:0031492",
  "gene_name": "Histone H3.3C",
  "gene": "UniProtKB:Q6NXT2",
  "term_label": "nucleosomal DNA binding",
  "gene_symbol": "H3-5"
}